peptidyl-arginine methylation, to asymmetrical-dimethyl arginine [GO:0019919] (biological process) Definition: The process of methylation of peptidyl-arginine to form peptidyl-N(omega),N(omega)-dimethyl-L-arginine. Relationships: is a type of GO:0035247 Also known as: peptidyl-arginine methylation, to unsymmetrical-dimethyl arginine Sources: RESID:AA0068, RESID:AA0069